{
  "gene_symbol": "CLRN2",
  "term_label": "Unknown biological process",
  "term_id": "UNKNOWN:0002",
  "gene": "UniProtKB:A0PK11",
  "gene_name": "Clarin-2"
}